{
  "gene": "UniProtKB:Q9UJ98",
  "term_id": "GO:0007062",
  "term_label": "sister chromatid cohesion",
  "gene_name": "Cohesin subunit SA-3",
  "gene_symbol": "STAG3"
}